{
  "gene_name": "C-C chemokine receptor type 2",
  "term_id": "GO:0005737",
  "gene_symbol": "CCR2",
  "gene": "UniProtKB:P41597",
  "term_label": "cytoplasm"
}